{
  "gene_symbol": "TRBV6-7",
  "gene_name": "Probable non-functional T cell receptor beta variable 6-7",
  "term_label": "plasma membrane",
  "gene": "UniProtKB:A0A0A0MS04",
  "term_id": "GO:0005886"
}